glycerophosphoinositol glycerophosphodiesterase activity [GO:0047395] (molecular function) Relationships: is a type of GO:0008081 Definition: Catalysis of the reaction: 1-(sn-glycero-3-phospho)-1D-myo-inositol + H2O = sn-glycerol 3-phosphate + myo-inositol + H+. Also known as: 1-(sn-glycero-3-phospho)-1D-myo-inositol glycerophosphohydrolase activity, sn-glycero(3)phosphoinositol glycerophosphohydrolase activity, sn-glycero-3-phospho-1-inositol glycerophosphohydrolase activity Sources: EC:3.1.4.44, RHEA:16501